{
  "gene": "UniProtKB:Q6UWE0",
  "gene_symbol": "LRSAM1",
  "term_id": "UNKNOWN:0002",
  "gene_name": "E3 ubiquitin-protein ligase LRSAM1",
  "term_label": "Unknown biological process"
}